{
  "gene": "UniProtKB:Q9ULI0",
  "term_label": "transcription initiation-coupled chromatin remodeling",
  "gene_name": "ATPase family AAA domain-containing protein 2B",
  "gene_symbol": "ATAD2B",
  "term_id": "GO:0045815"
}